early endosome membrane [GO:0031901] (cellular component) Sources: GOC:pz Definition: The lipid bilayer surrounding an early endosome. Subtypes: postsynaptic early endosome membrane [GO:0098896] Relationships: is a type of endosome membrane [GO:0010008]; is part of early endosome [GO:0005769]